{
  "term_id": "GO:0004364",
  "gene_symbol": "MGST1",
  "gene": "UniProtKB:P10620",
  "gene_name": "Microsomal glutathione S-transferase 1",
  "term_label": "glutathione transferase activity"
}